{
  "term_id": "GO:0004656",
  "gene_symbol": "P4HTM",
  "gene_name": "Transmembrane prolyl 4-hydroxylase",
  "term_label": "procollagen-proline 4-dioxygenase activity",
  "gene": "UniProtKB:Q9NXG6"
}